{
  "gene_name": "Potassium voltage-gated channel subfamily G member 1",
  "term_label": "membrane",
  "gene": "UniProtKB:Q9UIX4",
  "term_id": "GO:0016020",
  "gene_symbol": "KCNG1"
}